{
  "gene_symbol": "H2BC12",
  "term_label": "extracellular space",
  "gene": "UniProtKB:O60814",
  "gene_name": "Histone H2B type 1-K",
  "term_id": "GO:0005615"
}